{
  "term_label": "U1 snRNA 3'-end processing",
  "gene_symbol": "EXOSC8",
  "gene": "UniProtKB:Q96B26",
  "gene_name": "Exosome complex component RRP43",
  "term_id": "GO:0034473"
}